{
  "gene_name": "Embryonal Fyn-associated substrate",
  "term_label": "Unknown molecular function",
  "gene_symbol": "EFS",
  "gene": "UniProtKB:O43281",
  "term_id": "UNKNOWN:0001"
}